response to alkaline pH [GO:0010446] (BP) Subtypes: cellular response to alkaline pH [GO:0071469] Definition: Any process that results in a change in state or activity of a cell or an organism (in terms of movement, secretion, enzyme production, gene expression, etc.) as a result of a pH stimulus with pH > 7. pH is a measure of the acidity or basicity of an aqueous solution. Sources: GOC:go_curators, GOC:tb, Wikipedia:PH Also known as: response to alkalinity, response to basic pH Relationships: is a type of GO:0009268